mesonephric nephron tubule morphogenesis [GO:0061240] (biological process) Definition: The process in which the anatomical structures of a mesonephric nephron tubule are generated and organized. A mesonephric nephron tubule is an epithelial tube that is part of the mesonephric nephron, the functional part of the mesonephros. Relationships: is a type of mesonephric tubule morphogenesis [GO:0072171]; is part of mesonephric nephron morphogenesis [GO:0061228]; is part of mesonephric nephron tubule development [GO:0061242] Subtypes: mesonephric distal tubule morphogenesis [GO:0061273], mesonephric proximal tubule morphogenesis [GO:0061276] Sources: GOC:mtg_kidney_jan10